{
  "gene_symbol": "UTP18",
  "term_id": "UNKNOWN:0002",
  "term_label": "Unknown biological process",
  "gene_name": "U3 small nucleolar RNA-associated protein 18 homolog",
  "gene": "UniProtKB:Q9Y5J1"
}